{
  "term_label": "neuromuscular junction development",
  "term_id": "GO:0007528",
  "gene": "UniProtKB:P46934",
  "gene_symbol": "NEDD4",
  "gene_name": "E3 ubiquitin-protein ligase NEDD4"
}